{
  "term_id": "GO:0048306",
  "gene_name": "Protein S100-A8",
  "gene_symbol": "S100A8",
  "gene": "UniProtKB:P05109",
  "term_label": "calcium-dependent protein binding"
}